{
  "gene_name": "Choline_ethanolamine kinase",
  "term_label": "cytoplasm",
  "term_id": "GO:0005737",
  "gene_symbol": "CHKB",
  "gene": "UniProtKB:Q9Y259"
}